chloroplast avoidance movement [GO:0009903] (BP) Definition: The relocation process in which chloroplasts in photosynthetic cells avoid strong light and move away from it in order to preserve the photosynthetic machinery. References: PMID:11978863 Sources: GOC:tb Also known as: high-fluence-rate response Relationships: is a type of chloroplast relocation [GO:0009902]